nicotinamide mononucleotide transmembrane transport [GO:0035353] (biological process) Sources: GOC:bf, ISBN:0721662544 Relationships: is a type of nicotinamide mononucleotide transport [GO:0015890]; is a type of nucleotide transmembrane transport [GO:1901679] Also known as: nicotinamide mononucleotide membrane transport Definition: The process in which nicotinamide mononucleotide is transported across a membrane. Nicotinamide mononucleotide is a ribonucleotide in which the nitrogenous base, nicotinamide, is in beta-n-glycosidic linkage with the c-1 position of d-ribose. It is a constituent of NAD and NADP. Note: Note that this term is not intended for use in annotating lateral movement within membranes.